negative regulation of uredinium development [GO:0075282] (biological process) Relationships: is a type of negative regulation of spore-bearing organ development [GO:0075262]; is a type of regulation of uredinium development [GO:0075280]; negatively regulates uredinium development [GO:0075279] Sources: GOC:pamgo_curators Definition: Any process that stops, prevents, or reduces the frequency, rate or extent of uredinium development, a process that leads to the formation of a reddish, pustule-like structure formed by a rust fungus and consisting of uredospores.